alpha-beta intraepithelial T cell differentiation [GO:0002299] (biological process) Sources: GOC:add, ISBN:0781735149 Also known as: alpha-beta intraepithelial T lymphocyte differentiation, alpha-beta intraepithelial T-cell differentiation, alpha-beta intraepithelial T-lymphocyte differentiation, alpha-beta intraepithelial T cell development Relationships: is a type of alpha-beta T cell differentiation [GO:0046632] Definition: The process in which a precursor cell type acquires the specialized features of an alpha-beta intraepithelial T cell. Intraepithelial T cells are found among epithelial cells in mucosal areas and have distinct phenotypes and developmental pathways. Note: Note that immunologists typically use the word 'development' to refer to cells of B or T cell lineages undergoing the process that GO describes as 'cell differentiation'. Subtypes: CD8-positive, alpha-beta intraepithelial T cell differentiation [GO:0002300], CD4-positive, alpha-beta intraepithelial T cell differentiation [GO:0002301]